O-phosphoseryl-tRNA(Sec) selenium transferase activity [GO:0098621] (molecular function) Also known as: O-phospho-L-seryl-tRNA(Sec):L-selenocysteinyl-tRNA synthase, O-phosphoseryl-tRNA:selenocysteinyl-tRNA synthase, SepSecS, phosphoseryl-selenocysteinyl-tRNA selenium transferase activity Relationships: is a type of GO:0016785; is a type of catalytic activity, acting on a tRNA [GO:0140101] Definition: Catalysis of the reaction: O-phospho-L-seryl-tRNA(Sec) + selenophosphate + H2O = L-selenocysteinyl-tRNA(Sec) + 2 phosphate. References: PMID:17142313, PMID:19608919 Sources: RHEA:25041